{
  "gene_name": "Mucin-13",
  "gene": "UniProtKB:Q9H3R2",
  "term_label": "Unknown biological process",
  "term_id": "UNKNOWN:0002",
  "gene_symbol": "MUC13"
}